hatching [GO:0035188] (biological process) Definition: The emergence of an immature organism from a protective structure. Relationships: is a type of GO:0071684; is part of multicellular organism development [GO:0007275] Subtypes: GO:0001835 Sources: GOC:dgh, GOC:isa_complete, ISBN:0198612001